{
  "gene": "UniProtKB:E9PRG8",
  "gene_name": "Uncharacterized protein C11orf98",
  "gene_symbol": "C11orf98",
  "term_label": "Unknown biological process",
  "term_id": "UNKNOWN:0002"
}